{
  "term_id": "GO:0004674",
  "gene_name": "Inactive serine_threonine-protein kinase VRK3",
  "term_label": "protein serine/threonine kinase activity",
  "gene": "UniProtKB:Q8IV63",
  "gene_symbol": "VRK3"
}